{
  "gene": "UniProtKB:P62318",
  "term_label": "catalytic step 2 spliceosome",
  "gene_name": "Small nuclear ribonucleoprotein Sm D3",
  "term_id": "GO:0071013",
  "gene_symbol": "SNRPD3"
}